regulation of mitochondrial gene expression [GO:0062125] (biological process) References: PMID:28285835 Relationships: is_a regulation of gene expression [GO:0010468]; regulates mitochondrial gene expression [GO:0140053] Subtypes: regulation of mitochondrial translation [GO:0070129], GO:1903108 Definition: Any process that modulates the frequency, rate or extent of mitochondrial gene expression. Gene expression is the process in which a gene's coding sequence is converted into a mature gene product (protein or RNA).